{
  "gene_symbol": "RAB7B",
  "term_id": "UNKNOWN:0001",
  "gene_name": "Ras-related protein Rab-7b",
  "gene": "UniProtKB:Q96AH8",
  "term_label": "Unknown molecular function"
}